ciliary pro-basal body maturation [GO:0120311] (biological process) Definition: A process that is carried out at the cellular level which results in the conversion of an immature and partially assembled ciliary pro-basal body into a mature basal body that is capable of nucleating a cilium. References: PMID:26862392 Sources: GOC:ach, GOC:krc Also known as: flagellar pro-basal body maturation, flagellar probasal body maturation, pro-basal body maturation Relationships: is a type of GO:0022607; is a type of ciliary basal body organization [GO:0032053]